{
  "gene": "UniProtKB:A4D1P6",
  "term_id": "GO:0031902",
  "gene_symbol": "WDR91",
  "gene_name": "WD repeat-containing protein 91",
  "term_label": "late endosome membrane"
}